{
  "gene": "UniProtKB:Q9HBH0",
  "gene_name": "Rho-related GTP-binding protein RhoF",
  "gene_symbol": "RHOF",
  "term_id": "GO:0005886",
  "term_label": "plasma membrane"
}